{
  "gene_name": "Nuclear receptor-interacting protein 1",
  "term_label": "nuclear estrogen receptor binding",
  "gene": "UniProtKB:P48552",
  "term_id": "GO:0030331",
  "gene_symbol": "NRIP1"
}